{
  "gene_symbol": "WDR46",
  "term_label": "small-subunit processome",
  "term_id": "GO:0032040",
  "gene": "UniProtKB:O15213",
  "gene_name": "WD repeat-containing protein 46"
}